{
  "term_label": "potassium channel regulator activity",
  "gene": "UniProtKB:Q9NPA1",
  "term_id": "GO:0015459",
  "gene_symbol": "KCNMB3",
  "gene_name": "Calcium-activated potassium channel subunit beta-3"
}